xyloglucan:xyloglucosyl transferase activity [GO:0016762] (molecular function) Relationships: is a type of glucosyltransferase activity [GO:0046527] Definition: Catalysis of the cleavage of a beta-(1->4) bond in the backbone of a xyloglucan and transfers the xyloglucanyl segment on to O-4 of the non-reducing terminal glucose residue of an acceptor, which can be a xyloglucan or an oligosaccharide of xyloglucan. Also known as: endoxyloglucan transferase activity, endo-xyloglucan transferase activity, xyloglucan endotransglucosylase activity, xyloglucan:xyloglucan xyloglucanotransferase activity References: PMID:1400418, PMID:1554366 Sources: EC:2.4.1.207, GOC:ask